{
  "term_label": "maturation of LSU-rRNA from tricistronic rRNA transcript (SSU-rRNA, 5.8S rRNA, LSU-rRNA)",
  "gene_symbol": "FTSJ3",
  "term_id": "GO:0000463",
  "gene": "UniProtKB:Q8IY81",
  "gene_name": "pre-rRNA 2'-O-ribose RNA methyltransferase FTSJ3"
}